{
  "gene_symbol": "FGF3",
  "term_label": "fibroblast growth factor receptor binding",
  "term_id": "GO:0005104",
  "gene": "UniProtKB:P11487",
  "gene_name": "Fibroblast growth factor 3"
}